{
  "gene": "UniProtKB:P61313",
  "term_label": "cytoplasmic translation",
  "gene_symbol": "RPL15",
  "gene_name": "Large ribosomal subunit protein eL15",
  "term_id": "GO:0002181"
}